organelle assembly [GO:0070925] (biological process) Regulation: regulated by GO:1902115; negatively regulated by GO:1902116; positively regulated by positive regulation of organelle assembly [GO:1902117] Definition: The aggregation, arrangement and bonding together of a set of components to form an organelle. An organelle is an organized structure of distinctive morphology and function. Includes the nucleus, mitochondria, plastids, vacuoles, vesicles, ribosomes and the cytoskeleton. Excludes the plasma membrane. Sources: GOC:mah Relationships: is a type of organelle organization [GO:0006996]; is a type of cellular component assembly [GO:0022607] Subtypes: autophagosome assembly [GO:0000045], acrosome assembly [GO:0001675], phagolysosome assembly [GO:0001845], Nebenkern assembly [GO:0007287], female pronucleus assembly [GO:0035038], male pronucleus assembly [GO:0035039], multivesicular body assembly [GO:0036258], cilium assembly [GO:0060271], karyomere assembly [GO:0061471], Cvt vesicle assembly [GO:0071255], extracellular exosome assembly [GO:0071971], postsynaptic specialization assembly [GO:0098698], membraneless organelle assembly [GO:0140694], GO:0140923, gut granule assembly [GO:1902900], melanosome assembly [GO:1903232], spine apparatus assembly [GO:1905355], GO:1905556